response to homocysteine [GO:1905374] (biological process) Subtypes: cellular response to homocysteine [GO:1905375] References: PMID:26722473 Sources: GOC:TermGenie, GO_REF:0000071 Definition: Any process that results in a change in state or activity of a cell or an organism (in terms of movement, secretion, enzyme production, gene expression, etc.) as a result of a homocysteine stimulus. Also known as: response to 2-amino-4-mercaptobutyric acid, response to 2-amino-4-sulfanylbutanoic acid, response to Hcy Relationships: is a type of response to amino acid [GO:0043200]; is a type of response to nitrogen compound [GO:1901698]; is a type of response to oxygen-containing compound [GO:1901700]